cytoskeleton [GO:0005856] (cellular component) Relationships: is a type of intracellular membraneless organelle [GO:0043232] References: PMID:16959967, PMID:27419875 Sources: GOC:mah Definition: A cellular structure that forms the internal framework of eukaryotic and prokaryotic cells. The cytoskeleton includes intermediate filaments, microfilaments, microtubules, the microtrabecular lattice, and other structures characterized by a polymeric filamentous nature and long-range order within the cell. The various elements of the cytoskeleton not only serve in the maintenance of cellular shape but also have roles in other cellular functions, including cellular movement, cell division, endocytosis, and movement of organelles. Subtypes: GO:0014731, actin cytoskeleton [GO:0015629], microtubule cytoskeleton [GO:0015630], GO:0030863, GO:0032156, perinuclear theca [GO:0033011], intermediate filament cytoskeleton [GO:0045111], presynaptic cytoskeleton [GO:0099569], postsynaptic cytoskeleton [GO:0099571]